{
  "gene_symbol": "NFRKB",
  "gene": "UniProtKB:Q6P4R8",
  "term_label": "protease binding",
  "gene_name": "Nuclear factor related to kappa-B-binding protein",
  "term_id": "GO:0002020"
}